{
  "gene": "UniProtKB:P34931",
  "gene_name": "Heat shock 70 kDa protein 1-like",
  "term_label": "ATP hydrolysis activity",
  "term_id": "GO:0016887",
  "gene_symbol": "HSPA1L"
}